{
  "gene_name": "Short_branched chain specific acyl-CoA dehydrogenase, mitochondrial",
  "gene_symbol": "ACADSB",
  "gene": "UniProtKB:P45954",
  "term_label": "mitochondrion",
  "term_id": "GO:0005739"
}